{
  "gene_symbol": "TLR9",
  "gene": "UniProtKB:Q9NR96",
  "gene_name": "Toll-like receptor 9",
  "term_id": "GO:0007249",
  "term_label": "canonical NF-kappaB signal transduction"
}